L-glutamine import across plasma membrane [GO:1903803] (biological process) Relationships: is a type of glutamine transport [GO:0006868]; is a type of organic cation transport [GO:0015695]; is a type of amino acid import across plasma membrane [GO:0089718]; is_a L-alpha-amino acid transmembrane transport [GO:1902475] Regulation: regulated by regulation of L-glutamine import across plasma membrane [GO:1901034]; negatively regulated by negative regulation of L-glutamine import across plasma membrane [GO:1901035]; positively regulated by positive regulation of L-glutamine import across plasma membrane [GO:1901036] References: PMID:23895341 Sources: GOC:TermGenie, GO_REF:0000075 Definition: The directed movement of L-glutamine from outside of a cell, across the plasma membrane and into the cytosol. Also known as: L-glutamine import, L-glutamine import into cell, L-glutamine uptake